{
  "term_id": "GO:0007162",
  "gene": "UniProtKB:O60486",
  "term_label": "negative regulation of cell adhesion",
  "gene_symbol": "PLXNC1",
  "gene_name": "Plexin-C1"
}